{
  "gene_name": "V-type proton ATPase 116 kDa subunit a 1",
  "term_id": "GO:0007035",
  "gene": "UniProtKB:Q93050",
  "term_label": "vacuolar acidification",
  "gene_symbol": "ATP6V0A1"
}